{
  "gene_symbol": "TTLL3",
  "term_label": "flagellated sperm motility",
  "gene": "UniProtKB:Q9Y4R7",
  "term_id": "GO:0030317",
  "gene_name": "Tubulin monoglycylase TTLL3"
}